{
  "term_label": "site of double-strand break",
  "gene_name": "SMC5-SMC6 complex localization factor protein 2",
  "gene_symbol": "SLF2",
  "gene": "UniProtKB:Q8IX21",
  "term_id": "GO:0035861"
}